pollen sperm cell differentiation [GO:0048235] (biological process) Relationships: is a type of developmental process involved in reproduction [GO:0003006]; is a type of cell differentiation [GO:0030154]; is part of GO:0048232; is part of microgametogenesis [GO:0055046] Definition: The process in which a relatively unspecialized cell acquires specialized features of a haploid sperm cell within the plant gametophyte. Also known as: male gamete generation, sperm cell differentiation, male gametophyte sperm cell differentiation Sources: CL:0000366, GOC:jid, GOC:mtg_sensu